{
  "gene_symbol": "EPHA4",
  "gene": "UniProtKB:P54764",
  "term_label": "ephrin receptor signaling pathway",
  "gene_name": "Ephrin type-A receptor 4",
  "term_id": "GO:0048013"
}